{
  "gene_symbol": "OR9A2",
  "term_id": "UNKNOWN:0002",
  "gene_name": "Olfactory receptor 9A2",
  "gene": "UniProtKB:Q8NGT5",
  "term_label": "Unknown biological process"
}